{
  "term_label": "protein serine/threonine kinase activity",
  "gene_symbol": "VRK1",
  "gene_name": "Serine_threonine-protein kinase VRK1",
  "term_id": "GO:0004674",
  "gene": "UniProtKB:Q99986"
}